epidermal cell division [GO:0010481] (biological process) References: PMID:17450124 Also known as: hypodermal cell division Definition: Any process resulting in the physical partitioning and separation of an epidermal cell, any of the cells making up the epidermis, into daughter cells. Relationships: is a type of GO:0051301 Regulation: regulated by regulation of epidermal cell division [GO:0010482]